{
  "gene_name": "Keratin, type I cytoskeletal 23",
  "term_label": "cytoskeleton",
  "term_id": "GO:0005856",
  "gene": "UniProtKB:Q9C075",
  "gene_symbol": "KRT23"
}